{
  "gene_symbol": "SENP5",
  "gene_name": "Sentrin-specific protease 5",
  "term_id": "GO:0016926",
  "gene": "UniProtKB:Q96HI0",
  "term_label": "protein desumoylation"
}